{
  "gene": "UniProtKB:O75128",
  "term_label": "actin monomer binding",
  "term_id": "GO:0003785",
  "gene_name": "Protein cordon-bleu",
  "gene_symbol": "COBL"
}